RNA polymerase II CTD heptapeptide repeat T4 kinase activity [GO:0140835] (molecular function) Relationships: is a type of RNA polymerase II CTD heptapeptide repeat kinase activity [GO:0008353] Definition: Catalysis of the reaction: ATP + RNA polymerase II large subunit CTD heptapeptide repeat (consensus YSPTSPS) = ADP + H+ + RNA polymerase II large subunit phosphothreonine (position 4). Also known as: RNA polymerase II C-terminal domain T4 kinase activity References: PMID:28248323